{
  "gene": "UniProtKB:Q7RTM1",
  "gene_name": "Proton channel OTOP1",
  "term_id": "GO:0015252",
  "gene_symbol": "OTOP1",
  "term_label": "proton channel activity"
}